{
  "gene": "UniProtKB:Q7Z5G4",
  "term_id": "GO:0005795",
  "gene_name": "Golgin subfamily A member 7",
  "term_label": "Golgi stack",
  "gene_symbol": "GOLGA7"
}